UDP-N-acetylmuramoyl-tripeptide-D-alanyl-D-alanine ligase activity [GO:0047480] (molecular function) Note: Note that the enzyme UDP-N-acetylmuramoyl-tripeptide-D-alanyl-D-alanine ligase also has UDP-N-acetylmuramoylalanyl-D-glutamyl-2,6-diaminopimelate-D-alanyl-D-alanine ligase activity (GO:0008766). Relationships: is_a GO:0016881 Also known as: UDP-N-acetylmuramoylalanine-D-glutamyl-lysine-D-alanyl-D-alanine ligase activity, UDP-N-acetylmuramoylalanyl-tripeptide-D-alanyl-D-alanine ligase activity, MurF synthetase activity, UDP-MurNAc-L-Ala-D-Glu-L-Lys:D-Ala-D-Ala ligase activity, UDP-MurNAc-pentapeptide synthetase activity, UDP-N-acetylmuramoyl-L-alanyl-D-glutamyl-L-lysine:D-alanyl-D-alanine ligase (ADP-forming), UDP-N-acetylmuramoyl-L-alanyl-D-glutamyl-L-lysyl-D-alanyl-D-alanine synthetase activity, UDP-N-acetylmuramoyl-L-alanyl-D-glutamyl-meso-2,6-diaminopimeloyl-D-alanyl-D-alanine synthetase activity, UDP-N-acetylmuramoylalanine-D-glutamyl-lysine--D-alanyl-D-alanine ligase activity, UDP-N-acetylmuramoylalanyl-D-glutamyl-2,6-diaminopimelate--D-alanyl-D-alanine ligase activity, UDP-N-acetylmuramoylalanyl-D-glutamyl-lysine-D-alanyl-D-alanine ligase activity, UDPacetylmuramoylpentapeptide synthetase activity, uridine diphosphoacetylmuramoylpentapeptide synthetase activity Sources: EC:6.3.2.10 Definition: Catalysis of the reaction: UDP-N-acetylmuramoyl-L-alanyl-D-glutamyl-L-lysine + ATP + D-alanyl-D-alanine = phosphate + UDP-N-acetylmuramoyl-L-alanyl-D-glutamyl-L-lysyl-D-alanyl-D-alanine + ADP.